adhesion of symbiont to host epithelial cell [GO:0044651] (biological process) Definition: The attachment of a symbiont to a host epithelial cell via adhesion molecules, general stickiness etc., either directly or indirectly. References: PMID:10066176 Sources: GOC:jl Relationships: is a type of adhesion of symbiont to host cell [GO:0044650]